{
  "term_id": "GO:0005768",
  "gene": "UniProtKB:Q687X5",
  "gene_symbol": "STEAP4",
  "gene_name": "Metalloreductase STEAP4",
  "term_label": "endosome"
}